{
  "gene": "UniProtKB:Q96JB2",
  "term_id": "GO:0006891",
  "gene_name": "Conserved oligomeric Golgi complex subunit 3",
  "term_label": "intra-Golgi vesicle-mediated transport",
  "gene_symbol": "COG3"
}